hydroxyneurosporene-O-methyltransferase activity [GO:0043803] (molecular function) Definition: Catalysis of the reaction: demethylspheroidene + S-adenosyl-L-methionine = H+ + S-adenosyl-L-homocysteine + spheroidene. References: PMID:12664193, PMID:12770713, PMID:7358679 Sources: RHEA:30903 Also known as: 1-HO-carotenoid methylase, 1-hydroxycarotenoid O-methylase, 1-hydroxycarotenoid methylase, demethylspheroidene O-methyltransferase Relationships: is_a methyltransferase activity [GO:0008168]